4-hydroxycoumarin catabolic process [GO:1901883] (biological process) Definition: The chemical reactions and pathways resulting in the breakdown of 4-hydroxycoumarin. References: PMID:19757094 Sources: GOC:TermGenie Also known as: 4-hydroxycoumarin breakdown, 4-hydroxycoumarin catabolism, 4-hydroxycoumarin degradation Relationships: is a type of coumarin catabolic process [GO:0046226]